{
  "gene": "UniProtKB:Q8N8Z3",
  "term_label": "Unknown molecular function",
  "gene_name": "Putative uncharacterized protein DIP2C-AS1",
  "term_id": "UNKNOWN:0001",
  "gene_symbol": "DIP2C-AS1"
}